ribose-5-phosphate isomerase activity [GO:0004751] (molecular function) Also known as: 5-phosphoribose isomerase activity, D-ribose 5-phosphate isomerase activity, D-ribose-5-phosphate aldose-ketose-isomerase activity, D-ribose-5-phosphate ketol-isomerase activity, pentose phosphate isomerase (PPI), phosphopentoseisomerase activity, phosphopentosisomerase activity, phosphoriboisomerase activity, ribose 5-phosphate epimerase activity, ribose phosphate isomerase activity Definition: Catalysis of the reaction: aldehydo-D-ribose 5-phosphate = D-ribulose 5-phosphate. Sources: RHEA:14657 Relationships: is a type of intramolecular oxidoreductase activity, interconverting aldoses and ketoses [GO:0016861]